{
  "gene_name": "Trafficking protein particle complex subunit 3",
  "gene": "UniProtKB:O43617",
  "term_id": "GO:0030008",
  "gene_symbol": "TRAPPC3",
  "term_label": "TRAPP complex"
}